{
  "gene": "UniProtKB:Q9BQ04",
  "term_id": "GO:0016607",
  "gene_name": "RNA-binding protein 4B",
  "gene_symbol": "RBM4B",
  "term_label": "nuclear speck"
}